{
  "term_id": "GO:0071013",
  "gene_symbol": "MAGOH",
  "gene_name": "Protein mago nashi homolog",
  "gene": "UniProtKB:P61326",
  "term_label": "catalytic step 2 spliceosome"
}